{
  "gene_name": "Zinc finger protein 620",
  "gene_symbol": "ZNF620",
  "term_id": "GO:0000981",
  "gene": "UniProtKB:Q6ZNG0",
  "term_label": "DNA-binding transcription factor activity, RNA polymerase II-specific"
}